{
  "term_id": "GO:0005634",
  "gene": "UniProtKB:P62256",
  "term_label": "nucleus",
  "gene_symbol": "UBE2H",
  "gene_name": "Ubiquitin-conjugating enzyme E2 H"
}